{
  "gene_symbol": "ABCA7",
  "term_id": "GO:0034188",
  "gene": "UniProtKB:Q8IZY2",
  "term_label": "apolipoprotein A-I receptor activity",
  "gene_name": "Phospholipid-transporting ATPase ABCA7"
}